negative regulation of MHC class II biosynthetic process [GO:0045347] (biological process) Sources: GOC:go_curators Also known as: down regulation of MHC class II biosynthetic process, down-regulation of MHC class II biosynthetic process, downregulation of MHC class II biosynthetic process, negative regulation of MHC class II anabolism, negative regulation of MHC class II biosynthesis, negative regulation of MHC class II formation, negative regulation of MHC class II synthesis, negative regulation of major histocompatibility complex class II biosynthesis, negative regulation of major histocompatibility complex class II biosynthetic process, inhibition of MHC class II biosynthetic process Relationships: is a type of negative regulation of macromolecule biosynthetic process [GO:0010558]; is a type of regulation of MHC class II biosynthetic process [GO:0045346]; negatively regulates MHC class II biosynthetic process [GO:0045342] Definition: Any process that stops, prevents, or reduces the frequency, rate or extent of the chemical reactions and pathways resulting in the formation of MHC class II.